{
  "gene": "UniProtKB:Q8N103",
  "term_label": "Unknown cellular component",
  "gene_name": "T-cell activation Rho GTPase-activating protein",
  "term_id": "UNKNOWN:0003",
  "gene_symbol": "TAGAP"
}